{
  "term_label": "regulation of hydrogen peroxide metabolic process",
  "gene": "UniProtKB:Q86UR1",
  "term_id": "GO:0010310",
  "gene_symbol": "NOXA1",
  "gene_name": "NADPH oxidase activator 1"
}